{
  "term_id": "GO:0055120",
  "term_label": "striated muscle dense body",
  "gene": "UniProtKB:Q14331",
  "gene_symbol": "FRG1",
  "gene_name": "Protein FRG1"
}